{
  "gene_symbol": "FASTKD1",
  "gene": "UniProtKB:Q53R41",
  "gene_name": "FAST kinase domain-containing protein 1, mitochondrial",
  "term_label": "mitochondrial matrix",
  "term_id": "GO:0005759"
}